{
  "term_id": "GO:0060271",
  "gene_name": "Cilia- and flagella-associated protein 54",
  "gene_symbol": "CFAP54",
  "gene": "UniProtKB:Q96N23",
  "term_label": "cilium assembly"
}